{
  "term_label": "endoplasmic reticulum to Golgi vesicle-mediated transport",
  "gene": "UniProtKB:Q86SZ2",
  "gene_symbol": "TRAPPC6B",
  "term_id": "GO:0006888",
  "gene_name": "Trafficking protein particle complex subunit 6B"
}